MHC class I receptor activity [GO:0032393] (molecular function) Definition: Combining with an MHC class I protein complex to initiate a change in cellular activity. Class I here refers to classical class I molecules. Relationships: is a type of transmembrane signaling receptor activity [GO:0004888]; is a type of immune receptor activity [GO:0140375]; has part MHC class I protein binding [GO:0042288] Also known as: T cell receptor activity, alpha-beta T cell receptor activity, gamma-delta T cell receptor activity Subtypes: inhibitory MHC class I receptor activity [GO:0032396], activating MHC class I receptor activity [GO:0032397] Note: Note that this term is intended for annotation of gene products that act as receptors for MHC class I protein complexes, not for components of the MHC class I protein complexes themselves. Sources: GOC:add, ISBN:0781735149